{
  "term_id": "GO:0045599",
  "gene": "UniProtKB:Q9GZV5",
  "term_label": "negative regulation of fat cell differentiation",
  "gene_symbol": "WWTR1",
  "gene_name": "WW domain-containing transcription regulator protein 1"
}